{
  "term_label": "extracellular matrix structural constituent conferring tensile strength",
  "gene": "UniProtKB:P20908",
  "gene_name": "Collagen alpha-1(V) chain",
  "term_id": "GO:0030020",
  "gene_symbol": "COL5A1"
}